{
  "gene": "UniProtKB:Q147U1",
  "gene_symbol": "ZNF846",
  "gene_name": "Zinc finger protein 846",
  "term_label": "RNA polymerase II transcription regulatory region sequence-specific DNA binding",
  "term_id": "GO:0000977"
}